{
  "term_id": "UNKNOWN:0003",
  "term_label": "Unknown cellular component",
  "gene_symbol": "IFFO2",
  "gene_name": "Intermediate filament family orphan 2",
  "gene": "UniProtKB:Q5TF58"
}